{
  "gene_name": "Ras-related protein Rab-37",
  "term_id": "GO:0005794",
  "gene": "UniProtKB:Q96AX2",
  "term_label": "Golgi apparatus",
  "gene_symbol": "RAB37"
}